{
  "term_label": "plasma membrane",
  "gene": "UniProtKB:O95136",
  "term_id": "GO:0005886",
  "gene_symbol": "S1PR2",
  "gene_name": "Sphingosine 1-phosphate receptor 2"
}